CoA-transferase activity [GO:0008410] (molecular function) Subtypes: succinyl-CoA:3-oxo-acid CoA-transferase activity [GO:0008260], 4-hydroxybutyrate CoA-transferase activity [GO:0008411], L-carnitine CoA-transferase activity [GO:0008735], acetate CoA-transferase activity [GO:0008775], GO:0008814, propionate CoA-transferase activity [GO:0018729], glutaconate CoA-transferase activity [GO:0018730], formyl-CoA transferase activity [GO:0033608], succinyl-CoA:(R)-benzylsuccinate CoA-transferase activity [GO:0033877], bile-acid-CoA transferase activity [GO:0033881], acetyl-CoA:oxalate CoA-transferase [GO:0036412], 2-hydroxyisocaproate CoA-transferase activity [GO:0043712], cinnamoyl-CoA:phenyllactate CoA-transferase activity [GO:0043785], propionyl-CoA:succinate CoA-transferase activity [GO:0043821], succinyl-CoA:(R)-citramalate CoA-transferase activity [GO:0043961], succinate-hydroxymethylglutarate CoA-transferase activity [GO:0047369], succinate-citramalate CoA-transferase activity [GO:0047370], butyrate-acetoacetate CoA-transferase activity [GO:0047371], GO:0047569, 5-hydroxypentanoate CoA-transferase activity [GO:0047591], GO:0047775, malonate CoA-transferase activity [GO:0050078], succinyl-CoA:oxalate CoA-transferase [GO:0050161] Relationships: is a type of transferase activity, transferring sulphur-containing groups [GO:0016782] Definition: Catalysis of the transfer of a coenzyme A (CoA) group from one compound (donor) to another (acceptor). Sources: GOC:jl